{
  "gene_symbol": "TPPP",
  "term_id": "GO:0032273",
  "gene": "UniProtKB:O94811",
  "term_label": "positive regulation of protein polymerization",
  "gene_name": "Tubulin polymerization-promoting protein"
}